{
  "gene_name": "Protein Hikeshi",
  "gene": "UniProtKB:Q53FT3",
  "term_id": "GO:0030544",
  "term_label": "Hsp70 protein binding",
  "gene_symbol": "HIKESHI"
}